{
  "term_label": "Unknown molecular function",
  "gene_name": "Signal peptidase complex subunit 3",
  "gene": "UniProtKB:P61009",
  "term_id": "UNKNOWN:0001",
  "gene_symbol": "SPCS3"
}